{
  "gene": "UniProtKB:Q9BXT5",
  "gene_name": "Testis-expressed protein 15",
  "gene_symbol": "TEX15",
  "term_label": "male meiotic nuclear division",
  "term_id": "GO:0007140"
}